{
  "term_id": "GO:0006357",
  "gene_symbol": "ZNF587B",
  "gene": "UniProtKB:E7ETH6",
  "gene_name": "Zinc finger protein 587B",
  "term_label": "regulation of transcription by RNA polymerase II"
}